{
  "term_id": "GO:0042981",
  "gene_symbol": "MOAP1",
  "gene": "UniProtKB:Q96BY2",
  "term_label": "regulation of apoptotic process",
  "gene_name": "Modulator of apoptosis 1"
}